{
  "gene_name": "Coiled-coil domain-containing protein 8",
  "term_label": "3M complex",
  "gene": "UniProtKB:Q9H0W5",
  "term_id": "GO:1990393",
  "gene_symbol": "CCDC8"
}